negative regulation of lysosome organization [GO:1905672] (biological process) Relationships: is_a negative regulation of organelle organization [GO:0010639]; is a type of regulation of lysosome organization [GO:1905671]; negatively regulates lysosome organization [GO:0007040] References: PMID:25561470 Sources: GOC:TermGenie, GO_REF:0000058 Also known as: down regulation of lysosome organisation, down regulation of lysosome organization, down-regulation of lysosome organisation, down-regulation of lysosome organization, downregulation of lysosome organisation, downregulation of lysosome organization, negative regulation of lysosome organisation, inhibition of lysosome organisation, inhibition of lysosome organization, down regulation of lysosome organization and biogenesis, down-regulation of lysosome organization and biogenesis, downregulation of lysosome organization and biogenesis, inhibition of lysosome organization and biogenesis, negative regulation of lysosome organization and biogenesis Definition: Any process that stops, prevents or reduces the frequency, rate or extent of lysosome organization.